{
  "term_id": "GO:0006325",
  "gene_name": "Histone H2B type 1-K",
  "gene": "UniProtKB:O60814",
  "gene_symbol": "H2BC12",
  "term_label": "chromatin organization"
}